negative regulation of salivary gland boundary specification [GO:0045705] (biological process) Relationships: is_a GO:0045704; is_a GO:0051093; is a type of negative regulation of multicellular organismal process [GO:0051241]; negatively regulates salivary gland boundary specification [GO:0007432] Sources: GOC:go_curators, GOC:tb Subtypes: negative regulation of adult salivary gland boundary specification [GO:0045709], GO:0045710 Also known as: down regulation of salivary gland determination, down-regulation of salivary gland determination, downregulation of salivary gland determination, negative regulation of salivary gland determination, inhibition of salivary gland determination Definition: Any process that stops, prevents, or reduces the frequency, rate or extent of salivary gland determination.